{
  "gene_symbol": "BTK",
  "term_label": "plasma membrane",
  "gene_name": "Tyrosine-protein kinase BTK",
  "gene": "UniProtKB:Q06187",
  "term_id": "GO:0005886"
}